{
  "gene_name": "Allergin-1",
  "term_id": "GO:0004888",
  "gene_symbol": "MILR1",
  "term_label": "transmembrane signaling receptor activity",
  "gene": "UniProtKB:Q7Z6M3"
}